{
  "term_label": "alpha-1,3-mannosylglycoprotein 2-beta-N-acetylglucosaminyltransferase activity",
  "gene": "UniProtKB:P26572",
  "gene_symbol": "MGAT1",
  "gene_name": "Alpha-1,3-mannosyl-glycoprotein 2-beta-N-acetylglucosaminyltransferase",
  "term_id": "GO:0003827"
}